cell morphogenesis involved in neuron differentiation [GO:0048667] (biological process) Subtypes: auditory receptor cell morphogenesis [GO:0002093], photoreceptor cell morphogenesis [GO:0008594], neuromast hair cell morphogenesis [GO:0035678], GO:0060116 Sources: GOC:dph, GOC:tb Also known as: neuron morphogenesis involved in differentiation Relationships: is a type of cell morphogenesis [GO:0000902]; is part of neuron development [GO:0048666] Definition: The process in which the structures of a neuron are generated and organized. This process occurs while the initially relatively unspecialized cell is acquiring the specialized features of a neuron.